{
  "term_label": "Unknown molecular function",
  "gene_symbol": "ZCCHC2",
  "gene_name": "Zinc finger CCHC domain-containing protein 2",
  "term_id": "UNKNOWN:0001",
  "gene": "UniProtKB:Q9C0B9"
}